contractile vacuolar membrane [GO:0031164] (cellular component) Also known as: contractile vacuole membrane Definition: The lipid bilayer surrounding the contractile vacuole. Relationships: is a type of vacuolar membrane [GO:0005774]; is a type of cytoplasmic vesicle membrane [GO:0030659]; is part of contractile vacuole [GO:0000331] Sources: GOC:pg